{
  "gene_name": "Actin-related protein 2_3 complex subunit 4",
  "term_label": "Unknown molecular function",
  "gene_symbol": "ARPC4",
  "gene": "UniProtKB:P59998",
  "term_id": "UNKNOWN:0001"
}